{
  "gene": "UniProtKB:P46098",
  "term_label": "transmitter-gated monoatomic ion channel activity involved in regulation of postsynaptic membrane potential",
  "gene_symbol": "HTR3A",
  "gene_name": "5-hydroxytryptamine receptor 3A",
  "term_id": "GO:1904315"
}